transport-coupled glycolytic process through glucose-6-phosphate [GO:0061633] (biological process) Relationships: is_a glycolytic process through glucose-6-phosphate [GO:0061620]; is a type of GO:0061718; BFO_0000051 protein-N(PI)-phosphohistidine-glucose phosphotransferase system transporter activity [GO:0022855] Sources: GOC:dph Definition: The chemical reactions and pathways resulting in the breakdown of glucose into pyruvate, in which the glucose is converted to glucose-6-phosphate intermediate coupled to transmembrane transport.